radial spoke base 3 [GO:0120342] (CC) Relationships: is a type of radial spoke base [GO:0120339]; is part of radial spoke 3 [GO:0120335] Definition: The short portion of the radial spoke 3 (RS3 )that is directly anchored to the A microtubule of an axonemal microtubule doublet. References: PMID:22754630, PMID:25694453 Sources: GOC:krc